structural constituent of peritrophic membrane [GO:0016490] (MF) Definition: The action of a molecule that contributes to the structural integrity of the peritrophic membrane, a tubular sheath of cuticle that shields the epithelial cells of the midgut from the gut contents. An example of this is found in Drosophila melanogaster. Sources: GOC:mtg_sensu, ISBN:0879694238 Relationships: is a type of structural molecule activity [GO:0005198] Also known as: structural constituent of peritrophic matrix